right ventricular cardiac muscle tissue morphogenesis [GO:0003221] (biological process) Relationships: is a type of GO:0055010; is part of GO:0003215 Subtypes: right ventricular compact myocardium morphogenesis [GO:0003226], right ventricular trabecular myocardium morphogenesis [GO:0003227] Definition: The process in which the anatomical structures of the right cardiac ventricle muscle are generated and organized. Also known as: right ventricle myocardium morphogenesis Sources: GOC:mtg_heart